{
  "gene_symbol": "SLC6A19",
  "gene_name": "Sodium-dependent neutral amino acid transporter B(0)AT1",
  "gene": "UniProtKB:Q695T7",
  "term_id": "GO:0035725",
  "term_label": "sodium ion transmembrane transport"
}